{
  "gene_name": "Cysteine-rich secretory protein LCCL domain-containing 1",
  "gene": "UniProtKB:Q9H336",
  "term_label": "extracellular space",
  "term_id": "GO:0005615",
  "gene_symbol": "CRISPLD1"
}